chrorion micropyle [GO:0070825] (cellular component) References: PMID:18649270 Sources: GOC:cvs, GOC:mah Relationships: is a type of cellular anatomical structure [GO:0110165]; is part of egg chorion [GO:0042600] Definition: A single cone-shaped specialization that forms an opening in the egg chorion that allows sperm entry into the egg prior to fertilization.